{
  "term_id": "GO:0030041",
  "gene": "UniProtKB:O60610",
  "term_label": "actin filament polymerization",
  "gene_symbol": "DIAPH1",
  "gene_name": "Protein diaphanous homolog 1"
}